{
  "term_id": "GO:0030150",
  "gene_symbol": "DNAJC19",
  "gene_name": "Mitochondrial import inner membrane translocase subunit TIM14",
  "gene": "UniProtKB:Q96DA6",
  "term_label": "protein import into mitochondrial matrix"
}